{
  "gene_name": "Histidine--tRNA ligase, cytoplasmic",
  "gene": "UniProtKB:P12081",
  "term_id": "GO:0005829",
  "term_label": "cytosol",
  "gene_symbol": "HARS1"
}